anaerobic glycerol catabolic process [GO:0019588] (biological process) Definition: The anaerobic chemical reactions and pathways resulting in the breakdown of glycerol, yielding energy in the form of ATP. Relationships: is_a glycerol catabolic process [GO:0019563]; is a type of non-glycolytic fermentation [GO:0019662] Subtypes: GO:0019589 Sources: GOC:mah Also known as: glycerol fermentation